{
  "gene_name": "Tyrosine-protein phosphatase non-receptor type 12",
  "gene": "UniProtKB:Q05209",
  "gene_symbol": "PTPN12",
  "term_label": "cytoplasm",
  "term_id": "GO:0005737"
}